{
  "term_id": "UNKNOWN:0001",
  "gene_symbol": "CCDC197",
  "term_label": "Unknown molecular function",
  "gene_name": "Uncharacterized protein CCDC197",
  "gene": "UniProtKB:Q8NCU1"
}